{
  "gene": "UniProtKB:Q68DX3",
  "gene_symbol": "FRMPD2",
  "term_label": "bicellular tight junction assembly",
  "term_id": "GO:0070830",
  "gene_name": "FERM and PDZ domain-containing protein 2"
}